{
  "gene_name": "DNA dC-dU-editing enzyme APOBEC-3B",
  "gene_symbol": "APOBEC3B",
  "gene": "UniProtKB:Q9UH17",
  "term_label": "cytidine to uridine editing",
  "term_id": "GO:0016554"
}